{
  "gene_symbol": "C9orf78",
  "gene_name": "Splicing factor C9orf78",
  "term_label": "Unknown molecular function",
  "gene": "UniProtKB:Q9NZ63",
  "term_id": "UNKNOWN:0001"
}